positive regulation of interferon-beta production [GO:0032728] (biological process) Also known as: positive regulation of IFN-beta production, up regulation of interferon-beta production, up-regulation of interferon-beta production, upregulation of interferon-beta production, activation of interferon-beta production, positive regulation of interferon-beta biosynthetic process, positive regulation of interferon-beta secretion, stimulation of interferon-beta production References: PMID:15546383 Sources: GOC:mah Definition: Any process that activates or increases the frequency, rate, or extent of interferon-beta production. Relationships: is a type of positive regulation of type I interferon production [GO:0032481]; is a type of regulation of interferon-beta production [GO:0032648]; RO_0002213 GO:0032608